{
  "gene": "UniProtKB:P0CJ86",
  "gene_name": "Double homeobox protein 4-like protein 3",
  "term_label": "RNA polymerase II transcription regulatory region sequence-specific DNA binding",
  "term_id": "GO:0000977",
  "gene_symbol": "DUX4L3"
}